{
  "gene_symbol": "OPN1MW3",
  "gene_name": "Medium-wave-sensitive opsin 3",
  "gene": "UniProtKB:P0DN78",
  "term_id": "GO:0071482",
  "term_label": "cellular response to light stimulus"
}